{
  "term_label": "double-strand break repair",
  "gene_name": "BRISC and BRCA1-A complex member 1",
  "gene": "UniProtKB:Q9NWV8",
  "term_id": "GO:0006302",
  "gene_symbol": "BABAM1"
}